{
  "term_id": "GO:0043408",
  "gene_symbol": "PAK2",
  "term_label": "regulation of MAPK cascade",
  "gene": "UniProtKB:Q13177",
  "gene_name": "Serine_threonine-protein kinase PAK 2"
}